determination of dorsal/ventral asymmetry [GO:0048262] (biological process) Also known as: determination of dorsal-ventral asymmetry, determination of dorsoventral asymmetry, determination of adaxial/abaxial asymmetry Sources: GOC:jid Relationships: is a type of GO:0009855; is part of dorsal/ventral pattern formation [GO:0009953] Definition: Determination of asymmetry from the dorsal to the ventral side; as, the dorsoventral axis.